{
  "gene_name": "Interleukin-1 receptor-like 2",
  "term_id": "GO:0007166",
  "gene": "UniProtKB:Q9HB29",
  "term_label": "cell surface receptor signaling pathway",
  "gene_symbol": "IL1RL2"
}